{
  "gene": "UniProtKB:Q9H1C3",
  "gene_symbol": "GLT8D2",
  "term_id": "UNKNOWN:0001",
  "term_label": "Unknown molecular function",
  "gene_name": "Glycosyltransferase 8 domain-containing protein 2"
}